{
  "gene_name": "Ubiquitin carboxyl-terminal hydrolase 5",
  "gene": "UniProtKB:P45974",
  "term_label": "regulation of protein stability",
  "term_id": "GO:0031647",
  "gene_symbol": "USP5"
}